L-phenylalanine-pyruvate transaminase activity [GO:0047312] (molecular function) Sources: RHEA:13053 Relationships: is_a aromatic-amino-acid transaminase activity [GO:0008793] Definition: Catalysis of the reaction: pyruvate + L-phenylalanine = phenylpyruvate + L-alanine. Also known as: L-phenylalanine(L-histidine):pyruvate aminotransferase activity, phenylalanine (histidine) aminotransferase activity, phenylalanine(histidine) aminotransferase activity, phenylalanine(histidine) transaminase activity, phenylalanine(histidine):pyruvate aminotransferase activity, L-phenylalanine:pyruvate aminotransferase activity, L-phenylalanine:pyruvate transaminase activity, L-histidine:pyruvate aminotransferase activity, histidine aminotransferase activity, histidine:pyruvate aminotransferase activity